{
  "term_label": "plasma membrane",
  "term_id": "GO:0005886",
  "gene": "UniProtKB:A6NFX1",
  "gene_name": "Sphingosine-1-phosphate transporter MFSD2B",
  "gene_symbol": "MFSD2B"
}